{
  "term_label": "phosphatidylinositol-3,4-bisphosphate binding",
  "gene_name": "Pleckstrin homology domain-containing family A member 1",
  "gene_symbol": "PLEKHA1",
  "gene": "UniProtKB:Q9HB21",
  "term_id": "GO:0043325"
}